regulation of glutamate secretion, neurotransmission [GO:1903294] (biological process) Subtypes: negative regulation of glutamate secretion, neurotransmission [GO:1903295], positive regulation of glutamate secretion, neurotransmission [GO:1903296] References: PMID:16782817 Sources: GOC:TermGenie, GO_REF:0000058 Note: An example of this is Rab3gap1 in mouse (Q80UJ7) in PMID:16782817 inferred from mutant phenotype Definition: Any process that modulates the frequency, rate or extent of glutamate secretion, neurotransmission. Relationships: is a type of regulation of glutamate secretion [GO:0014048]; is a type of regulation of neurotransmitter secretion [GO:0046928]; is a type of regulation of synaptic transmission, glutamatergic [GO:0051966]; regulates glutamate secretion, neurotransmission [GO:0061535]